{
  "gene_name": "Unconventional myosin-XIX",
  "gene": "UniProtKB:Q96H55",
  "term_id": "GO:0006897",
  "gene_symbol": "MYO19",
  "term_label": "endocytosis"
}